{
  "gene": "UniProtKB:Q8IWX5",
  "gene_symbol": "SGPP2",
  "gene_name": "Sphingosine-1-phosphate phosphatase 2",
  "term_id": "GO:0042392",
  "term_label": "sphingosine-1-phosphate phosphatase activity"
}